negative regulation of dendrite extension [GO:1903860] (biological process) References: PMID:24898855 Sources: GOC:PARL, GOC:TermGenie, GOC:pad, GO_REF:0000058 Definition: Any process that stops, prevents or reduces the frequency, rate or extent of dendrite extension. Note: An example of this is Mul1 in mouse (UniProt ID Q8VCM5) in PMID:24898855 inferred from mutant phenotype. Also known as: down regulation of dendrite extension, down-regulation of dendrite extension, downregulation of dendrite extension, up regulation of dendrite retraction, up-regulation of dendrite retraction, inhibition of dendrite extension Relationships: is a type of negative regulation of cell growth [GO:0030308]; is a type of negative regulation of developmental growth [GO:0048640]; is a type of regulation of dendrite extension [GO:1903859]; negatively regulates GO:0097484